hair cycle [GO:0042633] (biological process) Relationships: is a type of GO:0042303 Regulation: regulated by GO:0042634; positively regulated by positive regulation of hair cycle [GO:0042635]; negatively regulated by negative regulation of hair cycle [GO:0042636] References: PMID:12230507 Sources: GOC:go_curators Definition: The cyclical phases of growth (anagen), regression (catagen), quiescence (telogen), and shedding (exogen) in the life of a hair; one of the collection or mass of filaments growing from the skin of an animal, and forming a covering for a part of the head or for any part or the whole of the body.